positive regulation of vascular associated smooth muscle cell proliferation [GO:1904707] (biological process) Relationships: is_a positive regulation of smooth muscle cell proliferation [GO:0048661]; is a type of GO:1904705; positively regulates vascular associated smooth muscle cell proliferation [GO:1990874] Definition: Any process that activates or increases the frequency, rate or extent of vascular smooth muscle cell proliferation. References: PMID:23246467 Sources: GOC:TermGenie, GO_REF:0000058 Also known as: positive regulation of VSMC proliferation, positive regulation of vascular smooth muscle cell proliferation, up regulation of VSMC proliferation, up regulation of vascular smooth muscle cell proliferation, up-regulation of VSMC proliferation, up-regulation of vascular smooth muscle cell proliferation, upregulation of VSMC proliferation, upregulation of vascular smooth muscle cell proliferation, activation of VSMC proliferation, activation of vascular smooth muscle cell proliferation